{
  "gene_symbol": "CNTN2",
  "term_id": "GO:0005886",
  "gene": "UniProtKB:Q02246",
  "gene_name": "Contactin-2",
  "term_label": "plasma membrane"
}